{
  "gene": "UniProtKB:Q9BW11",
  "term_label": "Unknown cellular component",
  "gene_symbol": "MXD3",
  "term_id": "UNKNOWN:0003",
  "gene_name": "Max dimerization protein 3"
}